{
  "gene_name": "Putative myc-like protein MYCLP1",
  "gene_symbol": "MYCLP1",
  "term_id": "GO:0000981",
  "term_label": "DNA-binding transcription factor activity, RNA polymerase II-specific",
  "gene": "UniProtKB:P12525"
}